{
  "term_label": "Unknown molecular function",
  "term_id": "UNKNOWN:0001",
  "gene": "UniProtKB:Q5H8C1",
  "gene_name": "FRAS1-related extracellular matrix protein 1",
  "gene_symbol": "FREM1"
}